{
  "term_id": "UNKNOWN:0003",
  "term_label": "Unknown cellular component",
  "gene": "UniProtKB:Q9BVG9",
  "gene_symbol": "PTDSS2",
  "gene_name": "Phosphatidylserine synthase 2"
}